{
  "term_label": "chromatin",
  "gene_name": "SWI_SNF-related matrix-associated actin-dependent regulator of chromatin subfamily A member 5",
  "gene_symbol": "SMARCA5",
  "gene": "UniProtKB:O60264",
  "term_id": "GO:0000785"
}